{
  "gene_name": "Immunoglobulin lambda variable 3-9",
  "gene": "UniProtKB:A0A075B6K5",
  "term_id": "GO:0019814",
  "term_label": "immunoglobulin complex",
  "gene_symbol": "IGLV3-9"
}